{
  "term_label": "plasma membrane",
  "gene_name": "Olfactory receptor 52I2",
  "gene_symbol": "OR52I2",
  "gene": "UniProtKB:Q8NH67",
  "term_id": "GO:0005886"
}